{
  "gene_name": "Cadherin-like and PC-esterase domain-containing protein 1",
  "term_id": "UNKNOWN:0002",
  "term_label": "Unknown biological process",
  "gene": "UniProtKB:A4D0V7",
  "gene_symbol": "CPED1"
}